dADP catabolic process [GO:0046057] (biological process) Relationships: is a type of purine deoxyribonucleotide catabolic process [GO:0009155]; is a type of purine deoxyribonucleoside diphosphate catabolic process [GO:0009184]; is a type of dADP metabolic process [GO:0046056] Sources: GOC:go_curators Definition: The chemical reactions and pathways resulting in the breakdown of dADP, deoxyadenosine diphosphate (2'-deoxyadenosine 5'-diphosphate). Also known as: dADP breakdown, dADP catabolism, dADP degradation